{
  "gene_symbol": "WDR36",
  "term_label": "small-subunit processome",
  "gene": "UniProtKB:Q8NI36",
  "term_id": "GO:0032040",
  "gene_name": "WD repeat-containing protein 36"
}